positive regulation of type B pancreatic cell apoptotic process [GO:2000676] (biological process) Sources: GOC:mtg_apoptosis, GOC:obol Definition: Any process that activates or increases the frequency, rate or extent of type B pancreatic cell apoptotic process. Relationships: is a type of positive regulation of epithelial cell apoptotic process [GO:1904037]; is a type of regulation of type B pancreatic cell apoptotic process [GO:2000674]; positively regulates type B pancreatic cell apoptotic process [GO:0097050] Also known as: positive regulation of pancreatic B cell apoptosis, positive regulation of pancreatic beta cell apoptosis, positive regulation of type B pancreatic cell apoptosis